{
  "gene_name": "Host cell factor 1",
  "gene_symbol": "HCFC1",
  "term_label": "transcription coactivator activity",
  "gene": "UniProtKB:P51610",
  "term_id": "GO:0003713"
}